{
  "term_label": "endoplasmic reticulum membrane",
  "term_id": "GO:0005789",
  "gene_symbol": "RETSAT",
  "gene_name": "All-trans-retinol 13,14-reductase",
  "gene": "UniProtKB:Q6NUM9"
}